{
  "term_id": "GO:1900229",
  "gene_name": "BPI fold-containing family A member 1",
  "gene": "UniProtKB:Q9NP55",
  "term_label": "negative regulation of single-species biofilm formation in or on host organism",
  "gene_symbol": "BPIFA1"
}